limonene 1,2-monooxygenase [NAD(P)H) activity [GO:0052601] (molecular function) Definition: Catalysis of the reaction: limonene + NAD(P)H + H+ + O2 = NAD(P)+ + H2O + limonene-1,2-epoxide. Can use either (4S)-limonene or (4R)-limonene as substrate. NADPH can act instead of NADH, although more slowly. Also known as: (S)-limonene,NAD(P)H:oxygen oxidoreductase activity, limonene 1,2-monooxygenase activity, (S)-limonene 1,2-monooxygenase activity, (-)-limonene 1,2-monooxygenase activity, (-)-limonene,NAD(P)H:oxygen oxidoreductase activity Relationships: is a type of GO:0016709; is a type of GO:0019113 References: PMID:8820855 Sources: EC:1.14.13.107